{
  "term_id": "GO:0000977",
  "gene": "UniProtKB:Q68EA5",
  "term_label": "RNA polymerase II transcription regulatory region sequence-specific DNA binding",
  "gene_symbol": "ZNF57",
  "gene_name": "Zinc finger protein 57"
}